{
  "term_label": "proton transmembrane transport",
  "gene_name": "Proton-coupled amino acid transporter 2",
  "gene": "UniProtKB:Q495M3",
  "term_id": "GO:1902600",
  "gene_symbol": "SLC36A2"
}